{
  "term_id": "UNKNOWN:0003",
  "term_label": "Unknown cellular component",
  "gene_symbol": "PRR29",
  "gene": "UniProtKB:P0C7W0",
  "gene_name": "Proline-rich protein 29"
}